{
  "term_id": "UNKNOWN:0001",
  "term_label": "Unknown molecular function",
  "gene_symbol": "TPD52L1",
  "gene_name": "Tumor protein D53",
  "gene": "UniProtKB:Q16890"
}